{
  "term_label": "Unknown biological process",
  "gene_name": "rRNA methyltransferase 3, mitochondrial",
  "gene": "UniProtKB:Q9HC36",
  "term_id": "UNKNOWN:0002",
  "gene_symbol": "MRM3"
}